{
  "gene": "UniProtKB:P42677",
  "term_id": "GO:0022627",
  "gene_name": "Small ribosomal subunit protein eS27",
  "gene_symbol": "RPS27",
  "term_label": "cytosolic small ribosomal subunit"
}